{
  "term_label": "endomembrane system",
  "gene_symbol": "RAB14",
  "term_id": "GO:0012505",
  "gene_name": "Ras-related protein Rab-14",
  "gene": "UniProtKB:P61106"
}